{
  "term_label": "Unknown cellular component",
  "term_id": "UNKNOWN:0003",
  "gene_name": "GDP-mannose 4,6 dehydratase",
  "gene": "UniProtKB:O60547",
  "gene_symbol": "GMDS"
}